{
  "gene_name": "Death-associated protein kinase 3",
  "term_id": "GO:0005634",
  "gene": "UniProtKB:O43293",
  "gene_symbol": "DAPK3",
  "term_label": "nucleus"
}